{
  "term_label": "regulation of transcription by RNA polymerase II",
  "term_id": "GO:0006357",
  "gene": "UniProtKB:A6NCS4",
  "gene_symbol": "NKX2-6",
  "gene_name": "Homeobox protein Nkx-2.6"
}